interleukin-15-mediated signaling pathway [GO:0035723] (biological process) Relationships: is a type of cytokine-mediated signaling pathway [GO:0019221]; is part of cellular response to interleukin-15 [GO:0071350] Also known as: IL-15-mediated signaling pathway, interleukin-15-mediated signalling pathway Definition: The series of molecular signals initiated by interleukin-15 binding to its receptor on the surface of a target cell, and ending with the regulation of a downstream cellular process, e.g. transcription. Sources: GOC:BHF, GOC:signaling